{
  "term_label": "response to nicotine",
  "term_id": "GO:0035094",
  "gene_name": "Neuronal acetylcholine receptor subunit alpha-4",
  "gene": "UniProtKB:P43681",
  "gene_symbol": "CHRNA4"
}